{
  "term_label": "Unknown cellular component",
  "term_id": "UNKNOWN:0003",
  "gene_symbol": "MAP3K15",
  "gene_name": "Mitogen-activated protein kinase kinase kinase 15",
  "gene": "UniProtKB:Q6ZN16"
}